candelabrum cell differentiation [GO:0021712] (biological process) Relationships: is a type of cell differentiation in hindbrain [GO:0021533]; is_a GO:0021953; is part of cerebellar Purkinje cell layer formation [GO:0021694] References: PMID:15157725 Sources: GOC:cls, GOC:dgh, GOC:dph, GOC:jid, GO_REF:0000021 Definition: The process in which neuroblasts acquire specialized structural and/or functional features that characterize the mature candelabrum cell. Differentiation includes the processes involved in commitment of a neuroblast to a candelabrum cell fate. A candelabrum cell is an inhibitory GABAergic interneuron found in the cerebellar cortex.